{
  "gene_symbol": "H2AC25",
  "gene": "UniProtKB:Q7L7L0",
  "term_label": "heterochromatin formation",
  "gene_name": "Histone H2A type 3",
  "term_id": "GO:0031507"
}